{
  "term_id": "GO:0003730",
  "gene": "UniProtKB:Q92615",
  "term_label": "mRNA 3'-UTR binding",
  "gene_symbol": "LARP4B",
  "gene_name": "La-related protein 4B"
}